propionyl-CoA catabolic process [GO:1902859] (biological process) Definition: The chemical reactions and pathways resulting in the breakdown of propionyl-CoA. References: PMID:15514053 Sources: GOC:TermGenie, GOC:mengo_curators, GO_REF:0000068 Relationships: is a type of GO:0036115; is a type of propionyl-CoA metabolic process [GO:1902858] Also known as: propionyl-CoA breakdown, propionyl-CoA catabolism, propionyl-CoA degradation